{
  "gene_name": "T cell receptor beta variable 18",
  "term_label": "Unknown molecular function",
  "term_id": "UNKNOWN:0001",
  "gene_symbol": "TRBV18",
  "gene": "UniProtKB:A0A087X0M5"
}